sphingolipid activator protein activity [GO:0030290] (molecular function) Also known as: saposin Sources: ISBN:0198506732 Definition: Any of a group of peptide cofactors of enzymes for the lysosomal degradation of sphingolipids. They stimulate various enzymes, including glucosylceramidase, galactosylceramidase, cerebroside-sulfatase, alpha-galactosidase, beta-galactosidase, and sphingomyelin phosphodiesterase. Relationships: is_a enzyme activator activity [GO:0008047]